host cell viral nucleoid [GO:0039643] (cellular component) Definition: The region of a host cell that contains the viral genome. Sources: GOC:bf, GOC:bm, GOC:jl Note: To annotate the region of the complete virus particle in which the viral genome is contained, instead use 'virion nucleoid ; GO:0039642'. Relationships: is a type of host intracellular part [GO:0033646]